{
  "gene_name": "Leucine-rich repeat LGI family member 3",
  "gene_symbol": "LGI3",
  "term_id": "GO:0008021",
  "gene": "UniProtKB:Q8N145",
  "term_label": "synaptic vesicle"
}